{
  "gene": "UniProtKB:O15067",
  "gene_symbol": "PFAS",
  "term_label": "purine nucleotide biosynthetic process",
  "gene_name": "Phosphoribosylformylglycinamidine synthase",
  "term_id": "GO:0006164"
}